{
  "gene_symbol": "ERVK-7",
  "gene": "UniProtKB:P63135",
  "term_id": "UNKNOWN:0002",
  "term_label": "Unknown biological process",
  "gene_name": "Endogenous retrovirus group K member 7 Pol protein"
}